{
  "term_label": "actin filament organization",
  "gene_name": "SH3 domain-containing protein 21",
  "gene_symbol": "SH3D21",
  "term_id": "GO:0007015",
  "gene": "UniProtKB:A4FU49"
}